{
  "term_label": "GTPase activity",
  "gene": "UniProtKB:P62834",
  "gene_symbol": "RAP1A",
  "gene_name": "Ras-related protein Rap-1A",
  "term_id": "GO:0003924"
}